{
  "term_label": "cell division site",
  "gene": "UniProtKB:Q16181",
  "gene_symbol": "SEPTIN7",
  "gene_name": "Septin-7",
  "term_id": "GO:0032153"
}